D-galactonate catabolic process [GO:0034194] (biological process) Definition: The chemical reactions and pathways resulting in the breakdown of D-galactonate, the anion of D-galactonic acid. Sources: GOC:ai, GOC:mah Also known as: D-galactonate breakdown, D-galactonate catabolism, D-galactonate degradation Relationships: is_a GO:0016052; is a type of galactonate catabolic process [GO:0019584]